{
  "gene": "UniProtKB:O60269",
  "term_label": "plasma membrane",
  "gene_symbol": "GPRIN2",
  "term_id": "GO:0005886",
  "gene_name": "G protein-regulated inducer of neurite outgrowth 2"
}